{
  "gene": "UniProtKB:O60826",
  "term_id": "GO:2000060",
  "gene_name": "Coiled-coil domain-containing protein 22",
  "gene_symbol": "CCDC22",
  "term_label": "positive regulation of ubiquitin-dependent protein catabolic process"
}